{
  "gene": "UniProtKB:O00622",
  "term_label": "positive regulation of cell differentiation",
  "term_id": "GO:0045597",
  "gene_name": "CCN family member 1",
  "gene_symbol": "CCN1"
}